{
  "term_id": "UNKNOWN:0001",
  "gene_name": "Protein C10",
  "term_label": "Unknown molecular function",
  "gene_symbol": "C12orf57",
  "gene": "UniProtKB:Q99622"
}